sodium channel activity [GO:0005272] (molecular function) Subtypes: voltage-gated sodium channel activity [GO:0005248], ligand-gated sodium channel activity [GO:0015280], bile acid-gated sodium channel activity [GO:0160228] Regulation: regulated by sodium channel regulator activity [GO:0017080]; negatively regulated by sodium channel inhibitor activity [GO:0019871] Definition: Enables the energy-independent facilitated diffusion of a sodium ion through a transmembrane aqueous pore or channel. Relationships: is a type of monoatomic cation channel activity [GO:0005261]; is a type of sodium ion transmembrane transporter activity [GO:0015081] Sources: GOC:BHF, GOC:mtg_transport, GOC:pr, ISBN:0815340729